{
  "gene": "UniProtKB:P0DPI3",
  "term_label": "Unknown cellular component",
  "term_id": "UNKNOWN:0003",
  "gene_name": "Centromere protein V-like protein 2",
  "gene_symbol": "CENPVL2"
}